{
  "gene_symbol": "DPYSL5",
  "term_id": "UNKNOWN:0002",
  "gene": "UniProtKB:Q9BPU6",
  "gene_name": "Dihydropyrimidinase-related protein 5",
  "term_label": "Unknown biological process"
}